{
  "gene_symbol": "BTNL10P",
  "gene": "UniProtKB:A8MVZ5",
  "gene_name": "Putative butyrophilin-like protein 10 pseudogene",
  "term_id": "GO:0050852",
  "term_label": "T cell receptor signaling pathway"
}